{
  "term_label": "signal transduction",
  "gene": "UniProtKB:Q8NGR6",
  "gene_symbol": "OR1B1",
  "gene_name": "Olfactory receptor 1B1",
  "term_id": "GO:0007165"
}